{
  "term_id": "GO:0030670",
  "gene_symbol": "PIP4P2",
  "gene": "UniProtKB:Q8N4L2",
  "term_label": "phagocytic vesicle membrane",
  "gene_name": "Type 2 phosphatidylinositol 4,5-bisphosphate 4-phosphatase"
}